{
  "gene": "UniProtKB:P43629",
  "term_label": "immune receptor activity",
  "gene_symbol": "KIR3DL1",
  "gene_name": "Killer cell immunoglobulin-like receptor 3DL1",
  "term_id": "GO:0140375"
}